{
  "gene_symbol": "NCOA1",
  "gene": "UniProtKB:Q15788",
  "term_label": "positive regulation of transcription by RNA polymerase II",
  "gene_name": "Nuclear receptor coactivator 1",
  "term_id": "GO:0045944"
}